response to cobalamin [GO:0033590] (biological process) Relationships: is a type of response to vitamin [GO:0033273]; is a type of response to nitrogen compound [GO:1901698]; is a type of response to oxygen-containing compound [GO:1901700] Subtypes: GO:0071297 Definition: Any process that results in a change in state or activity of a cell or an organism (in terms of movement, secretion, enzyme production, gene expression, etc.) as a result of a cobalamin (vitamin B12) stimulus. Also known as: response to vitamin B12 Sources: GOC:sl